{
  "term_label": "RNA nuclease activity",
  "term_id": "GO:0004540",
  "gene_name": "Ribonuclease 7",
  "gene_symbol": "RNASE7",
  "gene": "UniProtKB:Q9H1E1"
}